{
  "term_id": "GO:0005886",
  "gene_symbol": "FRMD8",
  "term_label": "plasma membrane",
  "gene": "UniProtKB:Q9BZ67",
  "gene_name": "FERM domain-containing protein 8"
}